12-beta-hydroxysteroid dehydrogenase (NADP+) activity [GO:0047521] (MF) Definition: Catalysis of the reaction: 3-alpha,7-alpha,12-beta-trihydroxy-5-beta-cholanate + NADP+ = 3-alpha,7-alpha-dihydroxy-12-oxo-5-beta-cholanate + H+ + NADPH. Sources: RHEA:21424 Also known as: 12beta-hydroxy steroid (nicotinamide adenine dinucleotide phosphate) dehydrogenase activity, 12beta-hydroxysteroid dehydrogenase activity, 12beta-hydroxysteroid:NADP+ 12-oxidoreductase activity, 3alpha,7alpha,12beta-trihydroxy-5beta-cholanate dehydrogenase activity Relationships: is a type of steroid dehydrogenase activity, acting on the CH-OH group of donors, NAD or NADP as acceptor [GO:0033764]